regulation of glycolytic process [GO:0006110] (biological process) Sources: GOC:go_curators Also known as: regulation of glycolysis involved in cellular glucose homeostasis Definition: Any process that modulates the frequency, rate or extent of glycolysis. Subtypes: negative regulation of glycolytic process [GO:0045820], GO:0045821, GO:1904538 Relationships: is a type of regulation of purine nucleotide catabolic process [GO:0033121]; is a type of GO:0043467; is a type of regulation of carbohydrate catabolic process [GO:0043470]; is a type of GO:1903578; regulates glycolytic process [GO:0006096]